{
  "term_label": "Unknown molecular function",
  "gene_symbol": "ANKRD28",
  "gene": "UniProtKB:O15084",
  "gene_name": "Serine_threonine-protein phosphatase 6 regulatory ankyrin repeat subunit A",
  "term_id": "UNKNOWN:0001"
}